tetrahydrofolylpolyglutamate metabolic process [GO:0046900] (biological process) Relationships: is a type of folic acid-containing compound metabolic process [GO:0006760] Definition: The chemical reactions and pathways involving tetrahydrofolylpolyglutamate, a folate derivative comprising tetrahydrofolate attached to a chain of glutamate residues. Sources: GOC:ai Subtypes: tetrahydrofolylpolyglutamate biosynthetic process [GO:0046901] Also known as: tetrahydrofolyl-[Glu](n) metabolic process, tetrahydrofolyl-[Glu](n) metabolism, tetrahydrofolylpolyglutamate metabolism